{
  "gene_name": "Myc proto-oncogene protein",
  "term_id": "GO:0000978",
  "gene_symbol": "MYC",
  "gene": "UniProtKB:P01106",
  "term_label": "RNA polymerase II cis-regulatory region sequence-specific DNA binding"
}